mitotic nuclear bridge stalk [GO:0140511] (cellular component) Relationships: is_a cellular anatomical structure [GO:0110165]; is part of GO:0140510 References: PMID:32848252 Definition: Either of the regions of a mitotic nuclear bridge proximal to the main portion of each daughter nucleus. The nuclear envelope in the stalk regions is depleted of nuclear pore complexes.